{
  "term_id": "GO:0030864",
  "gene_name": "Coactosin-like protein",
  "term_label": "cortical actin cytoskeleton",
  "gene_symbol": "COTL1",
  "gene": "UniProtKB:Q14019"
}